{
  "gene_name": "FKSG35",
  "term_label": "Unknown biological process",
  "gene_symbol": "FKSG35",
  "term_id": "UNKNOWN:0002",
  "gene": "UniProtKB:Q9BZC5"
}